{
  "gene_symbol": "JCHAIN",
  "term_label": "immunoglobulin receptor binding",
  "term_id": "GO:0034987",
  "gene_name": "Immunoglobulin J chain",
  "gene": "UniProtKB:P01591"
}